{
  "term_label": "endosome",
  "gene_symbol": "BACE2",
  "term_id": "GO:0005768",
  "gene_name": "Beta-secretase 2",
  "gene": "UniProtKB:Q9Y5Z0"
}